{
  "term_id": "GO:0001525",
  "term_label": "angiogenesis",
  "gene_symbol": "PLEKHG5",
  "gene": "UniProtKB:O94827",
  "gene_name": "Pleckstrin homology domain-containing family G member 5"
}